{
  "gene": "UniProtKB:Q8TAK5",
  "gene_name": "GA-binding protein subunit beta-2",
  "term_id": "GO:0000976",
  "term_label": "transcription cis-regulatory region binding",
  "gene_symbol": "GABPB2"
}